{
  "gene": "UniProtKB:Q9HBH9",
  "gene_name": "MAP kinase-interacting serine_threonine-protein kinase 2",
  "term_label": "nucleus",
  "gene_symbol": "MKNK2",
  "term_id": "GO:0005634"
}